{
  "gene_symbol": "A0A5F9ZH88",
  "term_id": "GO:0005886",
  "gene": "UniProtKB:A0A5F9ZH88",
  "term_label": "plasma membrane",
  "gene_name": "Immunoglobulin subtype domain-containing protein"
}